diaphragm development [GO:0060539] (biological process) Definition: The progression of the diaphragm over time from its initial formation to the mature structure. The diaphragm is a skeletal muscle that is responsible for contraction and expansion of the lungs. Sources: GOC:dph Relationships: is a type of skeletal muscle organ development [GO:0060538]; is part of respiratory system development [GO:0060541]